actin filament bundle of stereocilium [GO:0098860] (cellular component) References: PMID:15661519 Definition: A bundle of hundreds of cross-linked actin filaments (an actin cable), that is the supporting structure of a stereocilium. Filaments are oriented such that the the plus (barbed) ends are at the tip of the protrusion and are capped by a tip complex which bridges to the plasma membrane. Relationships: is a type of actin filament bundle of actin-based cell projection [GO:0098859]; BFO_0000050 stereocilium [GO:0032420]